{
  "term_id": "GO:0006355",
  "gene_symbol": "FOXN3",
  "gene_name": "Forkhead box protein N3",
  "gene": "UniProtKB:O00409",
  "term_label": "regulation of DNA-templated transcription"
}